regulation of macrophage derived foam cell differentiation [GO:0010743] (biological process) Sources: GOC:BHF, GOC:add, GOC:dph, GOC:tb Relationships: is a type of regulation of cell differentiation [GO:0045595]; RO_0002211 macrophage derived foam cell differentiation [GO:0010742] Subtypes: positive regulation of macrophage derived foam cell differentiation [GO:0010744], negative regulation of macrophage derived foam cell differentiation [GO:0010745] Definition: Any process that modulates the rate, frequency or extent of macrophage derived foam cell differentiation. Macrophage derived foam cell differentiation is the process in which a macrophage acquires the specialized features of a foam cell. A foam cell is a type of cell containing lipids in small vacuoles and typically seen in atherosclerotic lesions, as well as other conditions.